negative regulation of interleukin-26 production [GO:0032710] (biological process) Also known as: down regulation of interleukin-26 production, down-regulation of interleukin-26 production, downregulation of interleukin-26 production, negative regulation of IL-26 production, inhibition of interleukin-26 production, negative regulation of interleukin-26 biosynthetic process Sources: GOC:mah Relationships: is a type of negative regulation of cytokine production [GO:0001818]; is a type of regulation of interleukin-26 production [GO:0032670]; negatively regulates interleukin-26 production [GO:0032630] Definition: Any process that stops, prevents, or reduces the frequency, rate, or extent of interleukin-26 production.